{
  "term_id": "GO:0015095",
  "gene": "UniProtKB:Q9H8M5",
  "gene_name": "Metal transporter CNNM2",
  "term_label": "magnesium ion transmembrane transporter activity",
  "gene_symbol": "CNNM2"
}